{
  "term_label": "Unknown cellular component",
  "gene": "UniProtKB:O76042",
  "gene_name": "Putative uncharacterized protein encoded by ERC2-IT1",
  "gene_symbol": "ERC2-IT1",
  "term_id": "UNKNOWN:0003"
}